chitosome [GO:0045009] (cellular component) Definition: An intracellular membrane-bounded particle found in fungi and containing chitin synthase; it synthesizes chitin microfibrils. Chitin synthase activity exists in chitosomes and they are proposed to act as a reservoir for regulated transport of chitin synthase enzymes to the division septum. References: PMID:8970154 Sources: ISBN:0198506732 Relationships: is a type of cytoplasmic vesicle [GO:0031410]